{
  "term_id": "UNKNOWN:0003",
  "gene": "UniProtKB:Q69YG0",
  "gene_symbol": "TMEM42",
  "term_label": "Unknown cellular component",
  "gene_name": "Transmembrane protein 42"
}